{
  "term_id": "GO:0006633",
  "gene": "UniProtKB:P86397",
  "term_label": "fatty acid biosynthetic process",
  "gene_name": "Hydroxyacyl-thioester dehydratase type 2, mitochondrial",
  "gene_symbol": "HTD2"
}